{
  "gene_symbol": "LINC01558",
  "gene": "UniProtKB:Q9Y6Z2",
  "gene_name": "Uncharacterized protein encoded by LINC01558",
  "term_label": "Unknown molecular function",
  "term_id": "UNKNOWN:0001"
}